{
  "term_id": "GO:0008033",
  "gene": "UniProtKB:Q99575",
  "gene_name": "Ribonucleases P_MRP protein subunit POP1",
  "gene_symbol": "POP1",
  "term_label": "tRNA processing"
}